lens placode formation involved in camera-type eye formation [GO:0046619] (biological process) Sources: GOC:dph, GOC:mtg_sensu, GOC:sdb_2009, GOC:tb Definition: Establishment and formation of the optic placode, paired ectodermal placodes that become invaginated to form the embryonic lens vesicles. Also known as: optic placode formation in camera-type eye, optic placode formation involved in camera-style eye, optic placode formation involved in camera-type eye formation Relationships: is a type of lens placode formation [GO:0001743]; is part of embryonic camera-type eye formation [GO:0060900]